metanephric glomerulus vasculature morphogenesis [GO:0072276] (biological process) Sources: GOC:mtg_kidney_jan10 Definition: The process in which the anatomical structures of the metanephric glomerulus vasculature are generated and organized. The metanephric glomerulus vasculature is composed of the tubule structures that carry blood or lymph in the metanephric glomerulus. Relationships: is a type of GO:0072103; is part of metanephric glomerulus vasculature development [GO:0072239]; is part of metanephric glomerulus morphogenesis [GO:0072275]